sarcomere [GO:0030017] (cellular component) Sources: ISBN:0815316194 Definition: The repeating unit of a myofibril in a muscle cell, composed of an array of overlapping thick and thin filaments between two adjacent Z discs. Relationships: is a type of cellular anatomical structure [GO:0110165]; BFO_0000050 GO:0030016